{
  "gene": "UniProtKB:Q9BZJ4",
  "term_label": "Unknown molecular function",
  "gene_symbol": "SLC25A39",
  "term_id": "UNKNOWN:0001",
  "gene_name": "Probable mitochondrial glutathione transporter SLC25A39"
}